{
  "term_label": "transmembrane transporter activity",
  "term_id": "GO:0022857",
  "gene": "UniProtKB:Q86VL8",
  "gene_symbol": "SLC47A2",
  "gene_name": "Multidrug and toxin extrusion protein 2"
}